{
  "gene_name": "Golgin subfamily A member 6D",
  "term_id": "GO:0005801",
  "term_label": "cis-Golgi network",
  "gene": "UniProtKB:P0CG33",
  "gene_symbol": "GOLGA6D"
}